{
  "term_label": "antigen processing and presentation of endogenous peptide antigen via MHC class Ib",
  "gene_name": "UL16-binding protein 6",
  "gene_symbol": "RAET1L",
  "gene": "UniProtKB:Q5VY80",
  "term_id": "GO:0002476"
}